cellulose synthase (GDP-forming) activity [GO:0016761] (molecular function) Sources: EC:2.4.1.29 Also known as: GDP-glucose-beta-D-glucan glucosyltransferase activity, GDP-glucose-cellulose glucosyltransferase activity, GDP-glucose:1,4-beta-D-glucan 4-beta-D-glucosyltransferase activity, GDPglucose:1,4-beta-D-glucan 4-beta-D-glucosyltransferase activity, cellulose synthase (guanosine diphosphate-forming) activity, guanosine diphosphoglucose-1,4-beta-glucan glucosyltransferase activity, guanosine diphosphoglucose-cellulose glucosyltransferase activity Definition: Catalysis of the reaction: GDP-glucose + ((1,4)-beta-D-glucosyl)(n) = GDP + ((1,4)-beta-D-glucosyl)(n+1). Relationships: is a type of cellulose synthase activity [GO:0016759]